{
  "term_label": "plasma membrane",
  "gene": "UniProtKB:A0A5A6",
  "gene_symbol": "TRBV11-3",
  "term_id": "GO:0005886",
  "gene_name": "T cell receptor beta variable 11-3"
}